{
  "term_label": "Unknown molecular function",
  "gene_name": "Melanoma-associated antigen B17",
  "gene_symbol": "MAGEB17",
  "gene": "UniProtKB:A8MXT2",
  "term_id": "UNKNOWN:0001"
}